replication fork arrest [GO:0043111] (biological process) Definition: Any process that stops, prevents, or reduces the frequency, rate or extent of DNA replication by impeding the progress of the DNA replication fork. Replication fork arrest is one of the 'quality control' processes ensuring that DNA-dependent DNA replication occurs correctly. DNA replication fork arrest during DNA-dependent DNA replication is not known to occur outside of cases where a replication error needs to be prevented or corrected. References: PMID:14645529 Sources: GOC:jl, GOC:pr Subtypes: replication fork arrest at mating type locus [GO:0011000], replication fork arrest at rDNA repeats [GO:0031582], replication fork arrest involved in DNA replication termination [GO:0071807], replication fork arrest at tRNA locus [GO:0090001] Also known as: negative regulation of DNA replication at replication fork barrier, replication fork blocking, replication fork stalling Note: See also the biological process term 'site-specific replication termination ; GO:0071170' and its children. Relationships: is a type of DNA-templated DNA replication maintenance of fidelity [GO:0045005]; is a type of negative regulation of DNA-templated DNA replication [GO:2000104]